response to dithiothreitol [GO:0072720] (biological process) Definition: Any process that results in a change in state or activity of a cell or an organism (in terms of movement, secretion, enzyme production, gene expression, etc.) as a result of a dithiothreitol stimulus. Sources: GOC:mah Relationships: is_a response to oxygen-containing compound [GO:1901700] Also known as: response to 1,4-dithiothreitol, response to DTT Subtypes: cellular response to dithiothreitol [GO:0072721]